clathrin-dependent extracellular exosome endocytosis [GO:1990771] (biological process) References: PMID:24951588 Definition: The clathrin-mediated endocytosis of an extracellular exosome. Also known as: clathrin-mediated extracellular exosome endocytosis, exosome related Relationships: is a type of establishment of vesicle localization [GO:0051650]; is a type of clathrin-dependent endocytosis [GO:0072583]